{
  "gene_symbol": "MAF1",
  "term_label": "RNA polymerase III core binding",
  "term_id": "GO:0000994",
  "gene_name": "Repressor of RNA polymerase III transcription MAF1 homolog",
  "gene": "UniProtKB:Q9H063"
}